tissue development [GO:0009888] (biological process) Sources: ISBN:0471245208 Relationships: is a type of anatomical structure development [GO:0048856] Also known as: histogenesis and organogenesis, histogenesis Subtypes: GO:0002930, ectoderm development [GO:0007398], endoderm development [GO:0007492], mesoderm development [GO:0007498], digestive tract mesoderm development [GO:0007502], epidermis development [GO:0008544], GO:0009960, GO:0010087, stele development [GO:0010479], biomineral tissue development [GO:0031214], decidualization [GO:0046697], GO:0048383, meristem development [GO:0048507], mucosa-associated lymphoid tissue development [GO:0048537], bone marrow development [GO:0048539], lateral line development [GO:0048882], hypochord development [GO:0055016], GO:0060429, mesenchyme development [GO:0060485], muscle tissue development [GO:0060537], spongiotrophoblast layer development [GO:0060712], connective tissue development [GO:0061448], ganglion development [GO:0061548], integument development [GO:0080060], hypoblast development [GO:0090008], plant epidermis development [GO:0090558], cardiac jelly development [GO:1905072] Definition: The process whose specific outcome is the progression of a tissue over time, from its formation to the mature structure.